{
  "gene_symbol": "VAX1",
  "gene_name": "Ventral anterior homeobox 1",
  "term_id": "GO:0006357",
  "gene": "UniProtKB:Q5SQQ9",
  "term_label": "regulation of transcription by RNA polymerase II"
}